P-type calcium transporter activity [GO:0005388] (molecular function) Also known as: calcium pump, ATP-dependent calcium transmembrane transporter activity, calcium transmembrane transporter activity, phosphorylative mechanism, calcium transporting ATPase activity, calcium-transporting ATPase activity, calcium efflux ATPase, calcium-translocating P-type ATPase activity, sarco(endo)plasmic reticulum Ca2+-ATPase, ATPase-coupled calcium transmembrane transporter activity, Ca(2+)-transporting ATPase activity, Ca2+-transporting ATPase activity Sources: RHEA:18105 Relationships: is a type of calcium ion transmembrane transporter activity [GO:0015085]; is_a P-type ion transporter activity [GO:0015662]; is_a ATPase-coupled monoatomic cation transmembrane transporter activity [GO:0019829] Regulation: regulated by regulation of ATPase-coupled calcium transmembrane transporter activity [GO:1901894]; negatively regulated by negative regulation of ATPase-coupled calcium transmembrane transporter activity [GO:1901895]; positively regulated by positive regulation of ATPase-coupled calcium transmembrane transporter activity [GO:1901896] Subtypes: P-type calcium transporter activity involved in regulation of cardiac muscle cell membrane potential [GO:0086039], P-type calcium transporter activity involved in regulation of presynaptic cytosolic calcium ion concentration [GO:1905056], P-type calcium transporter activity involved in regulation of postsynaptic cytosolic calcium ion concentration [GO:1905059] Definition: Enables the transfer of a solute or solutes from one side of a membrane to the other according to the reaction: ATP + H2O + Ca2+(in) = ADP + phosphate + Ca2+(out).